{
  "gene_symbol": "MYO7B",
  "gene_name": "Unconventional myosin-VIIb",
  "term_label": "microvillus",
  "gene": "UniProtKB:Q6PIF6",
  "term_id": "GO:0005902"
}